1-butanol biosynthetic process [GO:0071271] (biological process) Definition: The chemical reactions and pathways resulting in the formation of 1-butanol, an alkyl primary alcohol with the formula C4H10O. Relationships: is a type of primary alcohol biosynthetic process [GO:0034309]; is a type of fatty alcohol biosynthetic process [GO:1903175] Also known as: butanol biosynthetic process, 1-butanol anabolism, 1-butanol biosynthesis, 1-butanol formation, 1-butanol synthesis, butan-1-ol biosynthetic process Subtypes: butyryl-CoA catabolic process to butanol [GO:0044582] Sources: GOC:ecd, GOC:mah